diencephalon morphogenesis [GO:0048852] (biological process) Relationships: is a type of anatomical structure morphogenesis [GO:0009653]; is part of diencephalon development [GO:0021536]; is part of forebrain morphogenesis [GO:0048853] Sources: GOC:cls, GOC:dgh, GOC:dph, GOC:jid, ISBN:0838580343 Definition: The process in which the anatomical structures of the diencephalon are generated and organized. The diencephalon is the paired caudal parts of the prosencephalon from which the thalamus, hypothalamus, epithalamus and subthalamus are derived; these regions regulate autonomic, visceral and endocrine function, and process information directed to the cerebral cortex.